{
  "term_label": "protein serine/threonine kinase activity",
  "term_id": "GO:0004674",
  "gene_name": "Cyclin-dependent kinase 20",
  "gene_symbol": "CDK20",
  "gene": "UniProtKB:Q8IZL9"
}